{
  "gene": "UniProtKB:Q96J84",
  "gene_symbol": "KIRREL1",
  "term_id": "GO:0050839",
  "term_label": "cell adhesion molecule binding",
  "gene_name": "Kin of IRRE-like protein 1"
}